{
  "gene_name": "NF-X1-type zinc finger protein NFXL1",
  "term_label": "regulation of DNA-templated transcription",
  "term_id": "GO:0006355",
  "gene_symbol": "NFXL1",
  "gene": "UniProtKB:Q6ZNB6"
}